{
  "gene": "UniProtKB:P62310",
  "term_id": "GO:0071011",
  "gene_name": "U6 snRNA-associated Sm-like protein LSm3",
  "gene_symbol": "LSM3",
  "term_label": "precatalytic spliceosome"
}